{
  "gene_symbol": "DLG2",
  "term_id": "GO:0035255",
  "term_label": "ionotropic glutamate receptor binding",
  "gene_name": "Disks large homolog 2",
  "gene": "UniProtKB:Q15700"
}